{
  "term_label": "phosphatidylserine catabolic process",
  "term_id": "GO:0006660",
  "gene_symbol": "ABHD16A",
  "gene": "UniProtKB:O95870",
  "gene_name": "Phosphatidylserine lipase ABHD16A"
}